{
  "gene": "UniProtKB:P00966",
  "term_label": "argininosuccinate metabolic process",
  "gene_name": "Argininosuccinate synthase",
  "gene_symbol": "ASS1",
  "term_id": "GO:0000053"
}